{
  "gene_name": "Lysosome membrane protein 2",
  "term_id": "GO:0006622",
  "gene": "UniProtKB:Q14108",
  "gene_symbol": "SCARB2",
  "term_label": "protein targeting to lysosome"
}